myosin II head/neck binding [GO:0032034] (molecular function) Definition: Binding to the head/neck region of a myosin II heavy chain. Relationships: is a type of GO:0032028; is a type of GO:0032038 Sources: GOC:mah